regulation of cytokinetic process [GO:0032954] (biological process) Relationships: is a type of regulation of cell cycle process [GO:0010564]; regulates cytokinetic process [GO:0032506] Subtypes: regulation of actomyosin contractile ring contraction [GO:0031991], regulation of cell septum assembly [GO:1901891], regulation of mitotic cytokinetic process [GO:1903436], regulation of cytokinesis, site selection [GO:2000073], GO:2000431 Sources: GOC:mah Definition: Any process that modulates the frequency, rate or extent of a cytokinetic process.